spheroidene biosynthetic process [GO:1901180] (biological process) Sources: GOC:TermGenie, GOC:yaf, UniPathway:UPA00683 Relationships: is a type of xanthophyll biosynthetic process [GO:0016123]; is_a ether biosynthetic process [GO:1901503] Definition: The chemical reactions and pathways resulting in the formation of spheroidene. Also known as: spheroidene anabolism, spheroidene biosynthesis, spheroidene formation, spheroidene synthesis